migrasome [GO:0140494] (cellular component) Relationships: is a type of intracellular membrane-bounded organelle [GO:0043231] References: PMID:25342562, PMID:31371827 Definition: A vesicular organelle that forms on retraction fibers behind migrating cells and mediates the release of cytoplasmic contents during cell migration.